{
  "term_id": "UNKNOWN:0001",
  "gene": "UniProtKB:Q6PKC3",
  "term_label": "Unknown molecular function",
  "gene_name": "Thioredoxin domain-containing protein 11",
  "gene_symbol": "TXNDC11"
}